{
  "gene_symbol": "DVL3",
  "gene_name": "Segment polarity protein dishevelled homolog DVL-3",
  "gene": "UniProtKB:Q92997",
  "term_id": "GO:0005109",
  "term_label": "frizzled binding"
}